{
  "gene_symbol": "GSR",
  "term_id": "GO:0045454",
  "gene_name": "Glutathione reductase, mitochondrial",
  "gene": "UniProtKB:P00390",
  "term_label": "cell redox homeostasis"
}